{
  "gene": "UniProtKB:Q96KX2",
  "gene_name": "F-actin-capping protein subunit alpha-3",
  "term_id": "GO:0051016",
  "term_label": "barbed-end actin filament capping",
  "gene_symbol": "CAPZA3"
}